copper incorporation into metallo-sulfur cluster [GO:0018427] (biological process) Also known as: copper incorporation into metallo-sulphur cluster Definition: The incorporation of copper into a metallo-sulfur cluster. Sources: GOC:ai Subtypes: copper incorporation into copper-sulfur cluster [GO:0018428] Relationships: is a type of metal incorporation into metallo-sulfur cluster [GO:0018282]